{
  "gene_symbol": "LDB2",
  "gene_name": "LIM domain-binding protein 2",
  "term_id": "GO:0005667",
  "gene": "UniProtKB:O43679",
  "term_label": "transcription regulator complex"
}